{
  "gene_name": "Cellular tumor antigen p53",
  "term_label": "chromatin",
  "gene_symbol": "TP53",
  "term_id": "GO:0000785",
  "gene": "UniProtKB:P04637"
}